intracellular calcium ion homeostasis [GO:0006874] (biological process) Definition: A homeostatic process involved in the maintenance of a steady state level of calcium ions within a cell. Subtypes: vacuolar calcium ion homeostasis [GO:0007036], GO:0032468, endoplasmic reticulum calcium ion homeostasis [GO:0032469], GO:0051480, GO:0051560 Relationships: is a type of intracellular monoatomic cation homeostasis [GO:0030003]; is a type of calcium ion homeostasis [GO:0055074] Also known as: regulation of calcium ion concentration, cellular calcium ion homeostasis Sources: GOC:ceb, GOC:mah